specification of posterior mesonephric tubule identity [GO:0072169] (biological process) Definition: The process in which the tubules of the posterior mesonephros acquire their identity. Relationships: is a type of anterior/posterior pattern specification involved in kidney development [GO:0072098]; is a type of specification of mesonephric tubule identity [GO:0072167]; is part of GO:0072166 Sources: GOC:mtg_kidney_jan10